{
  "gene": "UniProtKB:P47869",
  "term_id": "GO:0004890",
  "gene_name": "Gamma-aminobutyric acid receptor subunit alpha-2",
  "gene_symbol": "GABRA2",
  "term_label": "GABA-A receptor activity"
}